{
  "term_id": "GO:0030660",
  "gene_name": "Signal peptide peptidase-like 2C",
  "gene_symbol": "SPPL2C",
  "gene": "UniProtKB:Q8IUH8",
  "term_label": "Golgi-associated vesicle membrane"
}